{
  "term_id": "GO:0007265",
  "gene_name": "1-phosphatidylinositol 4,5-bisphosphate phosphodiesterase epsilon-1",
  "gene": "UniProtKB:Q9P212",
  "gene_symbol": "PLCE1",
  "term_label": "Ras protein signal transduction"
}